{
  "term_label": "Unknown molecular function",
  "gene": "UniProtKB:Q15032",
  "gene_name": "R3H domain-containing protein 1",
  "gene_symbol": "R3HDM1",
  "term_id": "UNKNOWN:0001"
}